{
  "gene_name": "GATOR complex protein WDR24",
  "gene_symbol": "WDR24",
  "term_label": "cytosol",
  "term_id": "GO:0005829",
  "gene": "UniProtKB:Q96S15"
}